{
  "term_id": "GO:0005549",
  "gene": "UniProtKB:Q8N0Y5",
  "term_label": "odorant binding",
  "gene_name": "Olfactory receptor 8I2",
  "gene_symbol": "OR8I2"
}